{
  "gene_name": "Hemoglobin subunit gamma-2",
  "gene": "UniProtKB:P69892",
  "term_id": "GO:0005344",
  "gene_symbol": "HBG2",
  "term_label": "oxygen carrier activity"
}